{
  "gene": "UniProtKB:Q92570",
  "gene_name": "Nuclear receptor subfamily 4 group A member 3",
  "term_id": "GO:0071376",
  "term_label": "cellular response to corticotropin-releasing hormone stimulus",
  "gene_symbol": "NR4A3"
}